{
  "term_id": "GO:0005739",
  "gene_name": "Creatine kinase U-type, mitochondrial",
  "gene": "UniProtKB:P12532",
  "gene_symbol": "CKMT1A",
  "term_label": "mitochondrion"
}